{
  "term_id": "UNKNOWN:0002",
  "gene_name": "Putative uncharacterized protein PAK6-AS1",
  "gene_symbol": "PAK6-AS1",
  "term_label": "Unknown biological process",
  "gene": "UniProtKB:Q8N910"
}